alanine-oxo-acid transaminase activity [GO:0047635] (MF) Definition: Catalysis of the reaction: L-alanine + a 2-oxo acid = pyruvate + an L-amino acid. Sources: EC:2.6.1.12, MetaCyc:ALANINE--OXO-ACID-AMINOTRANSFERASE-RXN Also known as: alanine-oxo-acid aminotransferase activity, L-alanine-alpha-keto acid aminotransferase activity, L-alanine:2-oxo-acid aminotransferase activity, alanine--oxo-acid aminotransferase activity, alanine-keto acid aminotransferase activity, alanine-oxo acid aminotransferase activity, leucine-alanine transaminase activity Relationships: is a type of transaminase activity [GO:0008483] Subtypes: L-alanine:2-oxoglutarate aminotransferase activity [GO:0004021]